{
  "term_label": "spermatogenesis",
  "term_id": "GO:0007283",
  "gene_name": "Androgen receptor",
  "gene_symbol": "AR",
  "gene": "UniProtKB:P10275"
}